{
  "gene": "UniProtKB:Q9NQX1",
  "term_label": "RNA polymerase II transcription regulatory region sequence-specific DNA binding",
  "gene_name": "PR domain zinc finger protein 5",
  "term_id": "GO:0000977",
  "gene_symbol": "PRDM5"
}